{
  "gene_name": "Ermin",
  "term_label": "regulation of cell shape",
  "gene_symbol": "ERMN",
  "gene": "UniProtKB:Q8TAM6",
  "term_id": "GO:0008360"
}